{
  "gene_symbol": "THOC6",
  "gene": "UniProtKB:Q86W42",
  "term_id": "GO:0000346",
  "term_label": "transcription export complex",
  "gene_name": "THO complex subunit 6 homolog"
}